{
  "term_label": "negative regulation of canonical Wnt signaling pathway",
  "term_id": "GO:0090090",
  "gene": "UniProtKB:Q8NBI3",
  "gene_symbol": "DRAXIN",
  "gene_name": "Draxin"
}